{
  "term_id": "GO:0008266",
  "gene": "UniProtKB:P0CB38",
  "gene_name": "Polyadenylate-binding protein 4-like",
  "term_label": "poly(U) RNA binding",
  "gene_symbol": "PABPC4L"
}